{
  "term_label": "Unknown molecular function",
  "gene_symbol": "FAM86C1P",
  "term_id": "UNKNOWN:0001",
  "gene_name": "Putative protein FAM86C1P",
  "gene": "UniProtKB:Q9NVL1"
}